{
  "term_id": "GO:0005765",
  "gene": "UniProtKB:Q53TN4",
  "gene_symbol": "CYBRD1",
  "term_label": "lysosomal membrane",
  "gene_name": "Plasma membrane ascorbate-dependent reductase CYBRD1"
}